{
  "gene_symbol": "ATG14",
  "gene_name": "Beclin 1-associated autophagy-related key regulator",
  "term_id": "GO:0000045",
  "term_label": "autophagosome assembly",
  "gene": "UniProtKB:Q6ZNE5"
}